{
  "gene": "UniProtKB:Q8N9V2",
  "gene_name": "Probable E3 ubiquitin-protein ligase TRIML1",
  "gene_symbol": "TRIML1",
  "term_label": "innate immune response",
  "term_id": "GO:0045087"
}